{
  "gene": "UniProtKB:O60224",
  "gene_name": "Protein SSX4",
  "term_label": "Unknown molecular function",
  "term_id": "UNKNOWN:0001",
  "gene_symbol": "SSX4"
}